postsynaptic cytoskeleton organization [GO:0099188] (biological process) Sources: GOC:dos Definition: A process that is carried out at the cellular level which results in the assembly, arrangement of constituent parts, or disassembly of cytoskeletal structures comprising cytoskeletal filaments and their associated proteins in the postsynaptic cytoskeleton. Relationships: is a type of GO:0007010; is part of postsynapse organization [GO:0099173] Subtypes: postsynaptic actin cytoskeleton organization [GO:0098974], postsynaptic intermediate filament cytoskeleton organization [GO:0099185], postsynaptic spectrin-associated cytoskeleton organization [GO:0099190]